{
  "gene_name": "Ubiquitin-conjugating enzyme E2 variant 2",
  "term_id": "GO:0031371",
  "gene": "UniProtKB:Q15819",
  "gene_symbol": "UBE2V2",
  "term_label": "ubiquitin conjugating enzyme complex"
}